{
  "term_id": "GO:0009898",
  "gene": "UniProtKB:P26045",
  "term_label": "cytoplasmic side of plasma membrane",
  "gene_name": "Tyrosine-protein phosphatase non-receptor type 3",
  "gene_symbol": "PTPN3"
}